positive regulation of innate immunity memory response [GO:1905682] (biological process) Also known as: up regulation of innate immunity memory response, up-regulation of innate immunity memory response, upregulation of innate immunity memory response, activation of innate immunity memory response Sources: GOC:TermGenie, GO_REF:0000058 Relationships: is a type of positive regulation of innate immune response [GO:0045089]; is a type of regulation of innate immunity memory response [GO:1905680]; RO_0002213 innate immunity memory response [GO:0090714] Definition: Any process that activates or increases the frequency, rate or extent of innate immunity memory response.